{
  "gene_name": "Large ribosomal subunit protein mL64",
  "term_label": "Unknown molecular function",
  "term_id": "UNKNOWN:0001",
  "gene_symbol": "GADD45GIP1",
  "gene": "UniProtKB:Q8TAE8"
}